G protein-coupled nucleotide receptor binding [GO:0031811] (molecular function) Subtypes: P2Y1 nucleotide receptor binding [GO:0031812], P2Y2 nucleotide receptor binding [GO:0031813], P2Y4 nucleotide receptor binding [GO:0031814], P2Y5 nucleotide receptor binding [GO:0031815], P2Y6 nucleotide receptor binding [GO:0031816], GO:0031817, P2Y9 nucleotide receptor binding [GO:0031818], P2Y10 nucleotide receptor binding [GO:0031819], P2Y11 nucleotide receptor binding [GO:0031820] Also known as: G-protein coupled nucleotide receptor binding, P2Y receptor binding, metabotropic nucleotide receptor binding, metabotropic nucleotide receptor ligand Relationships: is a type of G protein-coupled receptor binding [GO:0001664] Definition: Binding to a G protein-coupled (metabotropic) nucleotide receptor. Sources: GOC:mah, GOC:nln